perillic acid-CoA ligase (AMP-forming) activity [GO:0052686] (molecular function) Definition: Catalysis of the reaction: perillic acid + CoA-SH + ATP = H2O + AMP + diphosphate + perillyl-CoA. Also known as: perillyl-CoA synthetase activity, perillic acid:CoA ligase (AMP-forming) activity References: PMID:24952578 Sources: KEGG_REACTION:R06368 Relationships: is a type of GO:0016405; is a type of acid-thiol ligase activity [GO:0016878]